{
  "gene": "UniProtKB:Q8TF42",
  "term_label": "collagen-activated tyrosine kinase receptor signaling pathway",
  "term_id": "GO:0038063",
  "gene_name": "Ubiquitin-associated and SH3 domain-containing protein B",
  "gene_symbol": "UBASH3B"
}